{
  "gene_symbol": "TAS2R1",
  "term_label": "membrane",
  "gene": "UniProtKB:Q9NYW7",
  "gene_name": "Taste receptor type 2 member 1",
  "term_id": "GO:0016020"
}